{
  "gene_symbol": "CDC23",
  "term_id": "GO:0051301",
  "gene": "UniProtKB:Q9UJX2",
  "gene_name": "Cell division cycle protein 23 homolog",
  "term_label": "cell division"
}